{
  "term_label": "Unknown biological process",
  "gene_symbol": "UBTD2",
  "gene_name": "Ubiquitin domain-containing protein 2",
  "gene": "UniProtKB:Q8WUN7",
  "term_id": "UNKNOWN:0002"
}